{
  "term_label": "voltage-gated potassium channel complex",
  "gene_symbol": "KCNF1",
  "gene_name": "Potassium voltage-gated channel subfamily F member 1",
  "term_id": "GO:0008076",
  "gene": "UniProtKB:Q9H3M0"
}